cellular response to silicon dioxide [GO:0071251] (biological process) Also known as: cellular response to silica, cellular response to silox Sources: GOC:mah Definition: Any process that results in a change in state or activity of a cell (in terms of movement, secretion, enzyme production, gene expression, etc.) as a result of a silicon dioxide stimulus. Relationships: is_a response to silicon dioxide [GO:0034021]; is a type of cellular response to oxygen-containing compound [GO:1901701]